{
  "term_label": "Unknown biological process",
  "gene": "UniProtKB:Q9BXX3",
  "gene_symbol": "ANKRD30A",
  "gene_name": "Ankyrin repeat domain-containing protein 30A",
  "term_id": "UNKNOWN:0002"
}